{
  "gene_name": "Keratin-associated protein 19-3",
  "gene": "UniProtKB:Q7Z4W3",
  "term_id": "UNKNOWN:0002",
  "term_label": "Unknown biological process",
  "gene_symbol": "KRTAP19-3"
}